{
  "gene": "UniProtKB:Q92738",
  "term_label": "GTPase activator activity",
  "term_id": "GO:0005096",
  "gene_name": "USP6 N-terminal-like protein",
  "gene_symbol": "USP6NL"
}